{
  "gene_symbol": "PRSS50",
  "term_label": "threonine-type endopeptidase activity",
  "gene": "UniProtKB:Q9UI38",
  "term_id": "GO:0004298",
  "gene_name": "Probable threonine protease PRSS50"
}